coenzyme F420-1:gamma-L-glutamate ligase activity [GO:0052619] (molecular function) Relationships: is a type of GO:0043773 Sources: MetaCyc:RXN-8081 Definition: Catalysis of the reaction: GTP + L-glutamate + factor gamma-F420-1 = GDP + H+ + factor gamma-F420-2 + phosphate.